early phagosome [GO:0032009] (cellular component) Also known as: early phagocytic vesicle Relationships: is a type of phagocytic vesicle [GO:0045335] References: PMID:12388753 Sources: GOC:mah Definition: A membrane-bounded intracellular vesicle as initially formed upon the ingestion of particulate material by phagocytosis.